{
  "term_label": "Unknown molecular function",
  "gene": "UniProtKB:Q9NP74",
  "gene_name": "Palmdelphin",
  "term_id": "UNKNOWN:0001",
  "gene_symbol": "PALMD"
}